{
  "gene_name": "Glutamine-rich protein 2",
  "gene": "UniProtKB:Q9H0J4",
  "gene_symbol": "QRICH2",
  "term_id": "UNKNOWN:0001",
  "term_label": "Unknown molecular function"
}